{
  "gene": "UniProtKB:Q16650",
  "gene_symbol": "TBR1",
  "gene_name": "T-box brain protein 1",
  "term_id": "GO:0000981",
  "term_label": "DNA-binding transcription factor activity, RNA polymerase II-specific"
}